{
  "gene_symbol": "STX4",
  "gene": "UniProtKB:Q12846",
  "term_id": "GO:0005484",
  "gene_name": "Syntaxin-4",
  "term_label": "SNAP receptor activity"
}